{
  "term_label": "PAM complex, Tim23 associated import motor",
  "gene": "UniProtKB:Q9Y5T4",
  "gene_name": "DnaJ homolog subfamily C member 15",
  "term_id": "GO:0001405",
  "gene_symbol": "DNAJC15"
}